{
  "gene": "UniProtKB:P50607",
  "term_label": "Unknown molecular function",
  "gene_symbol": "TUB",
  "gene_name": "Tubby protein homolog",
  "term_id": "UNKNOWN:0001"
}